{
  "gene": "UniProtKB:Q5BKZ1",
  "gene_symbol": "ZNF326",
  "gene_name": "DBIRD complex subunit ZNF326",
  "term_label": "nucleus",
  "term_id": "GO:0005634"
}